{
  "term_id": "GO:0005634",
  "gene_name": "Zinc finger protein 395",
  "gene": "UniProtKB:Q9H8N7",
  "term_label": "nucleus",
  "gene_symbol": "ZNF395"
}